{
  "term_label": "SCF-dependent proteasomal ubiquitin-dependent protein catabolic process",
  "gene_name": "F-box_LRR-repeat protein 17",
  "gene": "UniProtKB:Q9UF56",
  "gene_symbol": "FBXL17",
  "term_id": "GO:0031146"
}